{
  "gene_symbol": "HSPB2",
  "gene_name": "Heat shock protein beta-2",
  "term_label": "nucleus",
  "gene": "UniProtKB:Q16082",
  "term_id": "GO:0005634"
}